GDP-mannose 4,6-dehydratase activity [GO:0008446] (molecular function) Also known as: GDP-D-mannose 4,6-dehydratase activity, GDP-D-mannose dehydratase activity, GDP-mannose 4,6-hydro-lyase (GDP-4-dehydro-6-deoxy-D-mannose-forming), GDP-mannose 4,6-hydro-lyase activity, GDPmannose 4,6-dehydratase activity, Gmd, guanosine 5'-diphosphate-D-mannose oxidoreductase activity, guanosine diphosphomannose 4,6-dehydratase activity, guanosine diphosphomannose oxidoreductase activity Definition: Catalysis of the reaction: GDP-alpha-D-mannose = GDP-4-dehydro-6-deoxy-alpha-D-mannose + H2O. Sources: EC:4.2.1.47, RHEA:23820 Relationships: is a type of GO:0016836